{
  "gene": "UniProtKB:Q8IVL5",
  "term_id": "GO:0019797",
  "gene_symbol": "P3H2",
  "gene_name": "Prolyl 3-hydroxylase 2",
  "term_label": "procollagen-proline 3-dioxygenase activity"
}